p-cumate 2,3-dioxygenase activity [GO:0018570] (molecular function) Relationships: is a type of oxidoreductase activity, acting on single donors with incorporation of molecular oxygen, incorporation of two atoms of oxygen [GO:0016702] Definition: Catalysis of the reaction: p-cumate + NADH + H+ + O2 = NAD+ + cis-2,3-dihydroxy-2,3-dihydro-p-cumate. Sources: RHEA:42344